trans-synaptic signaling by soluble gas, modulating synaptic transmission [GO:0099554] (biological process) Sources: GOC:dos Relationships: is a type of trans-synaptic signaling by soluble gas [GO:0099543]; is a type of trans-synaptic signaling, modulating synaptic transmission [GO:0099550] Note: Note that this term was created for the SynGO project, and will be obsoleted when the SynGO annotations are made in Noctua. Subtypes: trans-synaptic signaling by nitric oxide, modulating synaptic transmission [GO:0099555], trans-synaptic signaling by carbon monoxide, modulating synaptic transmission [GO:0099556] Definition: Cell-cell signaling between presynapse and postsynapse, via the release and reception of gaseous molecules, that modulates the synaptic transmission properties of the synapse.